{
  "term_id": "GO:0016567",
  "gene_name": "E3 ubiquitin-protein ligase RNF220",
  "gene": "UniProtKB:Q5VTB9",
  "gene_symbol": "RNF220",
  "term_label": "protein ubiquitination"
}